{
  "term_label": "plasma membrane",
  "gene_symbol": "RGS11",
  "gene": "UniProtKB:O94810",
  "term_id": "GO:0005886",
  "gene_name": "Regulator of G-protein signaling 11"
}